maturation of SSU-rRNA [GO:0030490] (biological process) Definition: Any process involved in the maturation of a precursor Small SubUnit (SSU) ribosomal RNA (rRNA) molecule into a mature SSU-rRNA molecule. Also known as: SSU-rRNA maturation, processing of 20S pre-rRNA Subtypes: maturation of SSU-rRNA from tricistronic rRNA transcript (SSU-rRNA, 5.8S rRNA, LSU-rRNA) [GO:0000462], GO:0000474, GO:0000489, maturation of SSU-rRNA from tricistronic rRNA transcript (SSU-rRNA, LSU-rRNA,5S) [GO:0002109] Relationships: is a type of rRNA processing [GO:0006364]; is part of ribosomal small subunit biogenesis [GO:0042274] Sources: GOC:curators